{
  "gene": "UniProtKB:Q92781",
  "term_label": "all-trans-retinol dehydrogenase (NAD+) activity",
  "term_id": "GO:0004745",
  "gene_name": "Retinol dehydrogenase 5",
  "gene_symbol": "RDH5"
}